{
  "gene_name": "Semaphorin-3A",
  "term_id": "GO:0038191",
  "gene": "UniProtKB:Q14563",
  "gene_symbol": "SEMA3A",
  "term_label": "neuropilin binding"
}